{
  "gene_symbol": "TPRX2",
  "term_id": "GO:0005634",
  "gene_name": "Tetrapeptide repeat homeobox protein 2",
  "gene": "UniProtKB:P0DV77",
  "term_label": "nucleus"
}